{
  "gene_symbol": "MYO1F",
  "gene_name": "Unconventional myosin-If",
  "term_id": "GO:0005886",
  "term_label": "plasma membrane",
  "gene": "UniProtKB:O00160"
}